glycogen binding [GO:2001069] (molecular function) Definition: Binding to glycogen. Sources: GOC:mengo_curators Also known as: animal starch binding, liver starch binding Relationships: is a type of polysaccharide binding [GO:0030247]